{
  "term_id": "UNKNOWN:0001",
  "term_label": "Unknown molecular function",
  "gene_symbol": "TAC3",
  "gene": "UniProtKB:Q9UHF0",
  "gene_name": "Tachykinin-3"
}